{
  "gene": "UniProtKB:O43278",
  "term_id": "GO:0060429",
  "term_label": "epithelium development",
  "gene_name": "Kunitz-type protease inhibitor 1",
  "gene_symbol": "SPINT1"
}